{
  "term_id": "GO:0008253",
  "gene": "UniProtKB:Q8TCD5",
  "gene_name": "5'(3')-deoxyribonucleotidase, cytosolic type",
  "term_label": "5'-nucleotidase activity",
  "gene_symbol": "NT5C"
}